{
  "term_id": "GO:0043025",
  "term_label": "neuronal cell body",
  "gene_symbol": "PDE1B",
  "gene": "UniProtKB:Q01064",
  "gene_name": "Dual specificity calcium_calmodulin-dependent 3',5'-cyclic nucleotide phosphodiesterase 1B"
}